exploration behavior [GO:0035640] (biological process) References: PMID:11682103, PMID:9767169 Sources: GOC:BHF, GOC:pr Note: For changes in locomotory behavior upon introduction to a novel environment, consider instead the child term: locomotory exploration behavior ; GO:0035641. Subtypes: locomotory exploration behavior [GO:0035641] Relationships: is a type of behavior [GO:0007610] Definition: The specific behavior of an organism in response to a novel environment or stimulus. Also known as: exploration behaviour, exploratory behavior, exploratory behaviour, open-field behavior